{
  "term_id": "GO:0000981",
  "gene_name": "Divergent paired-related homeobox",
  "term_label": "DNA-binding transcription factor activity, RNA polymerase II-specific",
  "gene_symbol": "DPRX",
  "gene": "UniProtKB:A6NFQ7"
}